{
  "gene_name": "Arf-GAP with SH3 domain, ANK repeat and PH domain-containing protein 2",
  "term_label": "Unknown biological process",
  "gene": "UniProtKB:O43150",
  "term_id": "UNKNOWN:0002",
  "gene_symbol": "ASAP2"
}